xanthine oxidase activity [GO:0004855] (molecular function) Relationships: is a type of oxidoreductase activity, acting on CH or CH2 groups, oxygen as acceptor [GO:0016727] Definition: Catalysis of the reaction: xanthine + H2O + O2 = urate + hydrogen peroxide. Sources: EC:1.17.3.2 Also known as: hypoxanthine-xanthine oxidase activity, xanthine oxidoreductase activity, Schardinger enzyme activity, schardinger enzyme, xanthine:O2 oxidoreductase activity, xanthine:oxygen oxidoreductase activity, xanthine:xanthine oxidase activity